{
  "term_id": "UNKNOWN:0001",
  "gene": "UniProtKB:P84157",
  "gene_name": "Matrix-remodeling-associated protein 7",
  "gene_symbol": "MXRA7",
  "term_label": "Unknown molecular function"
}